{
  "gene_name": "Ras and EF-hand domain-containing protein",
  "term_label": "GTP binding",
  "term_id": "GO:0005525",
  "gene": "UniProtKB:Q8IZ41",
  "gene_symbol": "RASEF"
}